{
  "term_id": "UNKNOWN:0003",
  "gene_name": "Putative uncharacterized protein SSBP3-AS1",
  "gene_symbol": "SSBP3-AS1",
  "gene": "UniProtKB:Q7Z2R9",
  "term_label": "Unknown cellular component"
}